{
  "gene_name": "Probable methyltransferase-like protein 24",
  "term_id": "UNKNOWN:0001",
  "gene": "UniProtKB:Q5JXM2",
  "term_label": "Unknown molecular function",
  "gene_symbol": "METTL24"
}